interleukin-17 receptor binding [GO:0030367] (molecular function) Sources: GOC:ai Relationships: is a type of cytokine receptor binding [GO:0005126] Also known as: IL-17, interleukin-17 receptor ligand Definition: Binding to an interleukin-17 receptor.